{
  "gene_symbol": "CIITA",
  "term_id": "UNKNOWN:0001",
  "gene": "UniProtKB:P33076",
  "term_label": "Unknown molecular function",
  "gene_name": "MHC class II transactivator"
}